cell migration to the midline involved in heart development [GO:0003318] (biological process) Definition: The orderly movement of a cell toward the midline that contributes to the progression of the heart over time. Subtypes: cardioblast migration to the midline involved in heart rudiment formation [GO:0003319], GO:0060975 Relationships: is a type of cell migration involved in heart development [GO:0060973] Sources: GOC:mtg_heart